{
  "gene_symbol": "OR13C5",
  "term_label": "detection of chemical stimulus involved in sensory perception of smell",
  "gene_name": "Olfactory receptor 13C5",
  "term_id": "GO:0050911",
  "gene": "UniProtKB:Q8NGS8"
}